{
  "gene": "UniProtKB:Q8IU85",
  "gene_name": "Calcium_calmodulin-dependent protein kinase type 1D",
  "gene_symbol": "CAMK1D",
  "term_label": "calmodulin binding",
  "term_id": "GO:0005516"
}